{
  "term_id": "GO:0005544",
  "gene_symbol": "SYT10",
  "term_label": "calcium-dependent phospholipid binding",
  "gene": "UniProtKB:Q6XYQ8",
  "gene_name": "Synaptotagmin-10"
}